{
  "gene_name": "Beta-2-microglobulin",
  "gene_symbol": "B2M",
  "gene": "UniProtKB:P61769",
  "term_label": "MHC class II protein complex binding",
  "term_id": "GO:0023026"
}